{
  "gene": "UniProtKB:Q99525",
  "term_id": "GO:0005634",
  "term_label": "nucleus",
  "gene_name": "Histone H4-like protein type G",
  "gene_symbol": "H4C7"
}